{
  "gene_name": "Solute carrier family 49 member A3",
  "term_label": "membrane",
  "gene_symbol": "SLC49A3",
  "term_id": "GO:0016020",
  "gene": "UniProtKB:Q6UXD7"
}